{
  "gene": "UniProtKB:P23468",
  "term_id": "GO:0007399",
  "gene_name": "Receptor-type tyrosine-protein phosphatase delta",
  "term_label": "nervous system development",
  "gene_symbol": "PTPRD"
}